{
  "gene_name": "Uncharacterized protein C12orf76",
  "gene_symbol": "C12orf76",
  "gene": "UniProtKB:Q8N812",
  "term_id": "UNKNOWN:0002",
  "term_label": "Unknown biological process"
}